{
  "term_label": "intraciliary transport particle B",
  "gene_name": "Intraflagellar transport protein 57 homolog",
  "gene": "UniProtKB:Q9NWB7",
  "term_id": "GO:0030992",
  "gene_symbol": "IFT57"
}